{
  "term_label": "Unknown cellular component",
  "gene_symbol": "POTEB",
  "gene": "UniProtKB:A0A0A6YYL3",
  "gene_name": "POTE ankyrin domain family member B",
  "term_id": "UNKNOWN:0003"
}